{
  "gene_name": "Xyloside xylosyltransferase 1",
  "term_id": "GO:0005789",
  "term_label": "endoplasmic reticulum membrane",
  "gene_symbol": "XXYLT1",
  "gene": "UniProtKB:Q8NBI6"
}